{
  "gene_symbol": "AGPAT4",
  "gene_name": "1-acyl-sn-glycerol-3-phosphate acyltransferase delta",
  "term_label": "1-acylglycerol-3-phosphate O-acyltransferase activity",
  "gene": "UniProtKB:Q9NRZ5",
  "term_id": "GO:0003841"
}